light-independent bacteriochlorophyll biosynthetic process [GO:0036070] (biological process) Also known as: light independent bacteriochlorophyll biosynthetic process, light-independent bacteriochlorophyll anabolism, light-independent bacteriochlorophyll biosynthesis, light-independent bacteriochlorophyll formation, light-independent bacteriochlorophyll synthesis Definition: The chemical reactions and pathways resulting in the formation of a bacteriochlorophyll, which occur in the absence of light. Bacteriochlorophylls are any of the chlorophylls of photosynthetic bacteria; they differ structurally from the chlorophylls of higher plants. Relationships: is a type of bacteriochlorophyll biosynthetic process [GO:0030494]; is a type of light-independent chlorophyll biosynthetic process [GO:0036068] References: PMID:12242396 Sources: GOC:yaf